{
  "term_label": "actin filament organization",
  "gene_symbol": "MARCKSL1",
  "gene": "UniProtKB:P49006",
  "gene_name": "MARCKS-related protein",
  "term_id": "GO:0007015"
}